Dsc E3 ubiquitin ligase complex assembly [GO:1990155] (biological process) References: PMID:23760507 Sources: GOC:mah Relationships: is a type of GO:0065003 Definition: The aggregation, arrangement and bonding together of a set of components to form a Dsc E3 ubiquitin ligase complex, an E3 ubiquitin ligase complex localized to the ER and Golgi membrane. Also known as: Dsc complex assembly